regulation of systemic arterial blood pressure by norepinephrine-epinephrine [GO:0001993] (biological process) Also known as: norepinephrine-epinephrine blood pressure regulation, noradrenaline-adrenaline regulation of blood pressure, norepinephrine-epinephrine blood pressure control Relationships: is a type of regulation of systemic arterial blood pressure mediated by a chemical signal [GO:0003044] Sources: ISBN:0721643949 Subtypes: positive regulation of blood pressure by epinephrine-norepinephrine [GO:0003321] Definition: The process in which the secretion of norepinephrine or epinephrine into the bloodstream modulates the force with which blood passes through the circulatory system.